{
  "gene_symbol": "KRT34",
  "term_label": "epithelial cell differentiation",
  "gene_name": "Keratin, type I cuticular Ha4",
  "gene": "UniProtKB:O76011",
  "term_id": "GO:0030855"
}